proteinogenic amino acid catabolic process [GO:0170040] (biological process) Relationships: is_a carboxylic acid catabolic process [GO:0046395]; is a type of proteinogenic amino acid metabolic process [GO:0170039] Definition: The chemical reactions and pathways resulting in the breakdown of any amino acid that is incorporated into protein naturally by ribosomal translation of mRNA, and that has a specific codon for translation from mRNA to protein. Subtypes: GO:0006527, L-asparagine catabolic process [GO:0006530], L-aspartate catabolic process [GO:0006533], L-glutamate catabolic process [GO:0006538], L-glutamine catabolic process [GO:0006543], glycine catabolic process [GO:0006546], GO:0006548, GO:0006550, GO:0006552, L-phenylalanine catabolic process [GO:0006559], GO:0006562, L-serine catabolic process [GO:0006565], L-threonine catabolic process [GO:0006567], GO:0006569, GO:0006572, L-valine catabolic process [GO:0006574], L-methionine catabolic process [GO:0009087], L-cysteine catabolic process [GO:0019448], L-lysine catabolic process [GO:0019477], L-alanine catabolic process [GO:0042853] Sources: GOC:ew Also known as: proteinogenic amino acid breakdown, proteinogenic amino acid catabolism, proteinogenic amino acid degradation